{
  "term_label": "Unknown biological process",
  "gene": "UniProtKB:Q8NH43",
  "term_id": "UNKNOWN:0002",
  "gene_symbol": "OR4L1",
  "gene_name": "Olfactory receptor 4L1"
}